{
  "gene": "UniProtKB:Q9H773",
  "gene_name": "dCTP pyrophosphatase 1",
  "term_id": "GO:0047840",
  "gene_symbol": "DCTPP1",
  "term_label": "dCTP diphosphatase activity"
}